glucan endo-1,2-beta-glucosidase activity [GO:0033913] (molecular function) Definition: Catalysis of the random hydrolysis of (1->2)-glucosidic linkages in (1->2)-beta-D-glucans. Relationships: is a type of beta-glucosidase activity [GO:0008422] Also known as: 1,2-beta-D-glucan glucanohydrolase activity, beta-D-1,2-glucanase activity, endo-(1->2)-beta-D-glucanase activity, endo-1,2-beta-glucanase activity Sources: EC:3.2.1.71